tRNA wobble guanine modification [GO:0002099] (biological process) Definition: The process in which a guanine at position 34 of a tRNA is post-transcriptionally modified. The wobble nucleoside of the tRNA sequence  (position 34) corresponds to the first position of the anticodon. Relationships: is a type of tRNA wobble base modification [GO:0002097] Subtypes: tRNA queuosine(34) biosynthetic process [GO:0008616] References: PMID:39600051 Sources: GOC:hjd